{
  "term_id": "GO:0006281",
  "gene_name": "PWWP domain-containing DNA repair factor 3A",
  "term_label": "DNA repair",
  "gene_symbol": "PWWP3A",
  "gene": "UniProtKB:Q2TAK8"
}